AP-3 adaptor complex [GO:0030123] (cellular component) References: PMID:10611976, PMID:21097499 Sources: GOC:mah Relationships: is a type of GO:0030119 Definition: A heterotetrameric AP-type membrane coat adaptor complex that consists of beta3, delta, mu3 and sigma3 subunits and is found associated with endosomal membranes. AP-3 does not appear to associate with clathrin in all organisms. In at least humans, the AP-3 complex can be heterogeneric due to the existence of multiple subunit isoforms encoded by different genes (beta3A and beta3B, mu3A and mu3B, and sigma3A and sigma3B).